{
  "term_label": "detection of mechanical stimulus involved in sensory perception of sound",
  "term_id": "GO:0050910",
  "gene": "UniProtKB:Q9UMZ3",
  "gene_symbol": "PTPRQ",
  "gene_name": "Phosphatidylinositol phosphatase PTPRQ"
}